{
  "gene_name": "Toll-like receptor 4",
  "term_id": "GO:0032497",
  "gene": "UniProtKB:O00206",
  "gene_symbol": "TLR4",
  "term_label": "detection of lipopolysaccharide"
}